{
  "gene": "UniProtKB:Q9HD42",
  "gene_name": "Charged multivesicular body protein 1a",
  "term_id": "GO:0032509",
  "term_label": "endosome transport via multivesicular body sorting pathway",
  "gene_symbol": "CHMP1A"
}